{
  "gene": "UniProtKB:P10696",
  "gene_name": "Alkaline phosphatase, germ cell type",
  "term_label": "Unknown biological process",
  "gene_symbol": "ALPG",
  "term_id": "UNKNOWN:0002"
}